{
  "gene_name": "Cyclin-dependent kinase 4",
  "term_id": "GO:0004693",
  "term_label": "cyclin-dependent protein serine/threonine kinase activity",
  "gene_symbol": "CDK4",
  "gene": "UniProtKB:P11802"
}